{
  "term_id": "UNKNOWN:0002",
  "term_label": "Unknown biological process",
  "gene_symbol": "NOP56",
  "gene_name": "Nucleolar protein 56",
  "gene": "UniProtKB:O00567"
}